{
  "term_id": "UNKNOWN:0001",
  "gene": "UniProtKB:Q5TZA2",
  "gene_name": "Rootletin",
  "term_label": "Unknown molecular function",
  "gene_symbol": "CROCC"
}